alveolar primary septum development [GO:0061143] (biological process) Definition: The progression of a primary alveolar septum over time, from its formation to the mature structure. A primary alveolar septum is a specialized epithelium that surrounds the saccule as it forms. Sources: GOC:dph Relationships: is a type of GO:0060428; is part of lung saccule development [GO:0060430]